protein localization to meiotic spindle midzone [GO:1903096] (biological process) Relationships: is a type of protein localization to meiotic spindle [GO:1905359] References: PMID:12707312 Sources: GOC:TermGenie, GOC:kmv, GO_REF:0000087 Definition: A process in which a protein is transported to, or maintained in, a location within a meiotic spindle midzone. Also known as: protein localisation in meiotic spindle midzone, protein localisation to meiotic spindle midzone, protein localization in meiotic spindle midzone